{
  "gene": "UniProtKB:Q2TBC4",
  "term_label": "Z disc",
  "gene_symbol": "PRICKLE4",
  "term_id": "GO:0030018",
  "gene_name": "Prickle-like protein 4"
}